quercetin 7-O-glucosyltransferase activity [GO:0080044] (molecular function) Definition: Catalysis of the transfer of a glucosyl group from UDP-glucose to the 7-hydroxy group of a quercetin molecule. References: PMID:15352060 Relationships: is a type of UDP-glucosyltransferase activity [GO:0035251]